exopolyphosphatase activity [GO:0004309] (molecular function) Sources: EC:3.6.1.11 Relationships: is_a pyrophosphatase activity [GO:0016462] Also known as: metaphosphatase activity, Gra-Pase activity, acid phosphoanhydride phosphohydrolase activity, exopolypase activity, polyphosphate phosphohydrolase activity Definition: Catalysis of the reaction: polyphosphate(n) + H2O = polyphosphate(n-1) + phosphate.